{
  "term_label": "G protein-coupled receptor signaling pathway",
  "gene": "UniProtKB:P01222",
  "gene_name": "Thyrotropin subunit beta",
  "gene_symbol": "TSHB",
  "term_id": "GO:0007186"
}